{
  "term_label": "synaptic transmission, GABAergic",
  "gene": "UniProtKB:A8MPY1",
  "gene_symbol": "GABRR3",
  "term_id": "GO:0051932",
  "gene_name": "Gamma-aminobutyric acid receptor subunit rho-3"
}